{
  "gene_symbol": "FABP1",
  "gene_name": "Fatty acid-binding protein, liver",
  "gene": "UniProtKB:P07148",
  "term_id": "GO:0005829",
  "term_label": "cytosol"
}